{
  "term_label": "axonal growth cone",
  "gene_symbol": "MYO9A",
  "gene": "UniProtKB:B2RTY4",
  "gene_name": "Unconventional myosin-IXa",
  "term_id": "GO:0044295"
}